hypoglossal nerve development [GO:0021566] (biological process) Relationships: is a type of cranial nerve development [GO:0021545] Also known as: cranial nerve XII development, CN XII development, cranial nerve 12 development Definition: The process whose specific outcome is the progression of the hypoglossal nerve over time, from its formation to the mature structure. This motor nerve innervates all the intrinsic and all but one of the extrinsic muscles of the tongue. Sources: GOC:cls, GOC:dgh, GOC:dph, GOC:jid, GO_REF:0000021